fear response [GO:0042596] (biological process) Relationships: is a type of multicellular organismal response to stress [GO:0033555] Also known as: physiological fear response Definition: The response of an organism to a perceived external threat. Subtypes: behavioral fear response [GO:0001662] Sources: GOC:go_curators Regulation: RO_0002211 by regulation of fear response [GO:1903365]; negatively regulated by negative regulation of fear response [GO:1903366]; positively regulated by GO:1903367